{
  "gene": "UniProtKB:Q495M3",
  "term_id": "GO:0015180",
  "gene_name": "Proton-coupled amino acid transporter 2",
  "term_label": "L-alanine transmembrane transporter activity",
  "gene_symbol": "SLC36A2"
}